homoserine metabolic process [GO:0009092] (biological process) Relationships: is a type of carboxylic acid metabolic process [GO:0019752] Also known as: homoserine metabolism Sources: GOC:go_curators, ISBN:0198506732 Subtypes: homoserine biosynthetic process [GO:0009090], homoserine catabolic process [GO:0009091], L-methionine biosynthetic process from L-homoserine via cystathionine [GO:0019279], L-methionine biosynthetic process from L-homoserine via O-acetyl-L-homoserine [GO:0019280], transsulfuration [GO:0019346] Definition: The chemical reactions and pathways involving homoserine, alpha-amino-gamma-hydroxybutyric acid, an intermediate in the biosynthesis of cystathionine, threonine and methionine.